histone locus body assembly [GO:0140167] (biological process) Relationships: is a type of GO:0030575; is a type of membraneless organelle assembly [GO:0140694] References: PMID:21576393, PMID:32401666 Definition: The aggregation, arrangement and bonding together of a set of components to form a histone locus body.